regulation of B cell tolerance induction [GO:0002661] (biological process) Definition: Any process that modulates the frequency, rate, or extent of B cell tolerance induction. Sources: GOC:add Also known as: regulation of B lymphocyte tolerance induction, regulation of B-cell tolerance induction, regulation of B-lymphocyte tolerance induction Relationships: is a type of regulation of tolerance induction [GO:0002643]; regulates B cell tolerance induction [GO:0002514] Subtypes: negative regulation of B cell tolerance induction [GO:0002662], positive regulation of B cell tolerance induction [GO:0002663], GO:0002670, regulation of B cell deletion [GO:0002867], regulation of central B cell tolerance induction [GO:0002895]